{
  "gene": "UniProtKB:P05000",
  "gene_name": "Interferon omega-1",
  "gene_symbol": "IFNW1",
  "term_id": "GO:0060337",
  "term_label": "type I interferon-mediated signaling pathway"
}